regulation of timing of exogen [GO:0051887] (biological process) Definition: Any process that modulates the frequency, rate or extent of timing of exogen, the shedding phase of the hair cycle. Sources: GOC:ai, GOC:pr Also known as: regulation of exogen Relationships: is a type of regulation of hair follicle maturation [GO:0048819]; regulates exogen [GO:0042638] Subtypes: positive regulation of timing of exogen [GO:0051888], negative regulation of timing of exogen [GO:0051889]